{
  "gene_name": "Coatomer subunit alpha",
  "gene": "UniProtKB:P53621",
  "term_label": "retrograde vesicle-mediated transport, Golgi to endoplasmic reticulum",
  "gene_symbol": "COPA",
  "term_id": "GO:0006890"
}